{
  "gene": "UniProtKB:Q60I27",
  "term_id": "GO:0016197",
  "gene_name": "ALS2 C-terminal-like protein",
  "gene_symbol": "ALS2CL",
  "term_label": "endosomal transport"
}